{
  "term_label": "Unknown molecular function",
  "gene": "UniProtKB:P59047",
  "term_id": "UNKNOWN:0001",
  "gene_name": "NACHT, LRR and PYD domains-containing protein 5",
  "gene_symbol": "NLRP5"
}